regulation of protein kinase C signaling [GO:0090036] (BP) Sources: GOC:dph, GOC:tb Also known as: regulation of protein kinase C signaling cascade, regulation of protein kinase C signalling cascade Relationships: is a type of regulation of intracellular signal transduction [GO:1902531]; regulates protein kinase C signaling [GO:0070528] Definition: Any process that modulates the frequency, rate, or extent of a series of reactions, mediated by the intracellular serine/threonine kinase protein kinase C, which occurs as a result of a single trigger reaction or compound. Subtypes: positive regulation of protein kinase C signaling [GO:0090037], GO:0090038